{
  "gene_symbol": "DEFB125",
  "gene": "UniProtKB:Q8N687",
  "term_label": "Unknown cellular component",
  "term_id": "UNKNOWN:0003",
  "gene_name": "Beta-defensin 125"
}